peptidyltransferase activity [GO:0000048] (molecular function) Definition: Catalysis of the reaction: peptidyl-tRNA(1) + aminoacyl-tRNA(2) = tRNA(1) + peptidylaminoacyl-tRNA(2). This reaction is catalyzed by a ribozyme. References: PMID:11433365, PMID:9242921 Relationships: is a type of aminoacyltransferase activity [GO:0016755]; is a type of GO:0140096; is a type of catalytic activity, acting on a tRNA [GO:0140101]